{
  "gene_symbol": "MESP2",
  "gene_name": "Mesoderm posterior protein 2",
  "term_label": "RNA polymerase II cis-regulatory region sequence-specific DNA binding",
  "gene": "UniProtKB:Q0VG99",
  "term_id": "GO:0000978"
}